{
  "term_label": "dendrite",
  "term_id": "GO:0030425",
  "gene_name": "Huntingtin",
  "gene": "UniProtKB:P42858",
  "gene_symbol": "HTT"
}